{
  "gene_name": "FYVE, RhoGEF and PH domain-containing protein 4",
  "term_id": "GO:0005085",
  "term_label": "guanyl-nucleotide exchange factor activity",
  "gene": "UniProtKB:Q96M96",
  "gene_symbol": "FGD4"
}